peptidyl-proline 3-dioxygenase activity [GO:0031544] (molecular function) Relationships: is_a peptidyl-proline dioxygenase activity [GO:0031543] Subtypes: procollagen-proline 3-dioxygenase activity [GO:0019797] Sources: GOC:mah Definition: Catalysis of the reaction: peptidyl L-proline + 2-oxoglutarate + O2 = peptidyl trans-3-hydroxy-L-proline + succinate + CO2.